peptide-methionine (R)-S-oxide reductase activity [GO:0033743] (molecular function) Definition: Catalysis of the reaction: L-methionyl-[protein] + [thioredoxin]-disulfide + H2O = L-methionyl-(R)-S-oxide-[protein] + [thioredoxin]-dithiol. Sources: RHEA:24164 Relationships: is a type of oxidoreductase activity, acting on a sulfur group of donors, disulfide as acceptor [GO:0016671]; is a type of GO:0140096 Also known as: methionine S-oxide reductase activity, methionine sulfoxide reductase activity, protein-methionine-R-oxide reductase activity, methionine sulfoxide reductase B activity, MsrB, PilB, SelR, SelX, methionine S-oxide reductase (R-form oxidizing) activity, pMRsr, pMSR, peptide-methionine:thioredoxin-disulfide S-oxidoreductase [methionine (R)-S-oxide-forming] activity, selenoprotein R